{
  "term_label": "DNA-binding transcription factor activity, RNA polymerase II-specific",
  "gene_symbol": "NFYB",
  "gene_name": "Nuclear transcription factor Y subunit beta",
  "gene": "UniProtKB:P25208",
  "term_id": "GO:0000981"
}